{
  "gene_name": "Brefeldin A-inhibited guanine nucleotide-exchange protein 3",
  "gene": "UniProtKB:Q5TH69",
  "term_id": "UNKNOWN:0003",
  "gene_symbol": "ARFGEF3",
  "term_label": "Unknown cellular component"
}